initiation of primordial ovarian follicle growth [GO:0001544] (biological process) Definition: Increase in size of primordial follicles including proliferation and shape changes of granulosa and/or theca cells until oocyte is surrounded by one layer of cuboidal shaped granulosa cells (primary follicle). Sources: https://www.ncbi.nlm.nih.gov/books/NBK279054/ Relationships: is a type of ovulation cycle process [GO:0022602]; is part of ovarian follicle development [GO:0001541]